positive regulation of antimicrobial peptide production [GO:0002225] (BP) Also known as: antimicrobial peptide induction, up regulation of antimicrobial peptide production, up-regulation of antimicrobial peptide production, upregulation of antimicrobial peptide production, activation of antimicrobial peptide production, stimulation of antimicrobial peptide production Definition: Any process that activates or increases the frequency, rate, or extent of antimicrobial peptide production. Relationships: is a type of positive regulation of production of molecular mediator of immune response [GO:0002702]; is a type of positive regulation of antimicrobial humoral response [GO:0002760]; is a type of regulation of antimicrobial peptide production [GO:0002784]; positively regulates antimicrobial peptide production [GO:0002775] Subtypes: positive regulation of antimicrobial peptide secretion [GO:0002796], positive regulation of antibacterial peptide production [GO:0002803], GO:0002804, positive regulation of antimicrobial peptide biosynthetic process [GO:0002807] References: PMID:11807545 Sources: GOC:add